3-oxosteroid 1-dehydrogenase activity [GO:0047571] (molecular function) Sources: EC:1.3.99.4 Definition: Catalysis of the reaction: a 3-oxosteroid + acceptor = a 3-oxo-D1-steroid + reduced acceptor. Also known as: 1-ene-dehydrogenase activity, 3-ketosteroid-1-en-dehydrogenase activity, 3-ketosteroid-delta1-dehydrogenase activity, 3-oxosteroid delta1-dehydrogenase activity, 3-oxosteroid:(2,6-dichlorphenolindophenol) delta1-oxidoreductase activity, 3-oxosteroid:(acceptor) delta1-oxidoreductase activity, 3-oxosteroid:acceptor delta1-oxidoreductase activity, 4-en-3-oxosteroid:(acceptor)-1-en-oxido-reductase activity, delta1-dehydrogenase activity, delta1-steroid reductase activity Relationships: is a type of GO:0033765